pyridoxal transmembrane transporter activity [GO:0031925] (molecular function) Definition: Enables the transfer of pyridoxal from one side of a membrane to the other. Pyridoxal, 3-hydroxy-5-(hydroxymethyl)-2-methyl-4-pyridinecarboxaldehyde, is one of the vitamin B6 compounds. Pyridoxal, pyridoxamine and pyridoxine are collectively known as vitamin B6, and are efficiently converted to the biologically active form of vitamin B6, pyridoxal phosphate. Sources: GOC:mah Relationships: is a type of transmembrane transporter activity [GO:0022857]; is part of pyridoxal transmembrane transport [GO:1903090] Also known as: pyridoxal transporter activity